{
  "gene": "UniProtKB:Q8NHZ8",
  "term_id": "GO:0070979",
  "term_label": "protein K11-linked ubiquitination",
  "gene_name": "Anaphase-promoting complex subunit CDC26",
  "gene_symbol": "CDC26"
}